unicellular trichome apex [GO:0090552] (cellular component) Definition: A cell projection part that is the apical most portion of a unicellular trichome. Sources: GOC:PO_curators, PO:0025537 Relationships: is_a cellular anatomical structure [GO:0110165]; is part of cell projection [GO:0042995]